{
  "gene_symbol": "A0A8I5KXM2",
  "gene_name": "Uncharacterized protein",
  "term_id": "UNKNOWN:0001",
  "term_label": "Unknown molecular function",
  "gene": "UniProtKB:A0A8I5KXM2"
}